{
  "term_id": "UNKNOWN:0002",
  "gene_symbol": "USP22",
  "gene": "UniProtKB:Q9UPT9",
  "term_label": "Unknown biological process",
  "gene_name": "Ubiquitin carboxyl-terminal hydrolase 22"
}